actomyosin contractile ring maturation [GO:0031566] (biological process) Subtypes: mitotic actomyosin contractile ring maturation [GO:1902406] Definition: The cellular process in which the contractile ring cytokinetic ring attains its fully functional state. References: PMID:25451933 Sources: GOC:vw Relationships: is a type of cellular component maintenance [GO:0043954]; is a type of GO:0044837 Also known as: actomyosin contractile ring maintenance, cytokinesis, contractile ring maintenance